regulation of protein autoubiquitination [GO:1902498] (biological process) Definition: Any process that modulates the frequency, rate or extent of protein autoubiquitination. Also known as: regulation of protein auto-ubiquitination, regulation of protein auto-ubiquitinylation, regulation of protein autoubiquitinylation, regulation of protein self-ubiquitination, regulation of protein self-ubiquitinylation Relationships: is a type of regulation of protein ubiquitination [GO:0031396]; regulates protein autoubiquitination [GO:0051865] Subtypes: positive regulation of protein autoubiquitination [GO:1902499], negative regulation of protein autoubiquitination [GO:1905524] References: PMID:24069405 Sources: GOC:TermGenie, GOC:rb